positive regulation of transforming growth factor beta receptor signaling pathway [GO:0030511] (biological process) Definition: Any process that activates or increases the frequency, rate or extent of TGF-beta receptor signaling pathway activity. Sources: GOC:go_curators Relationships: is a type of regulation of transforming growth factor beta receptor signaling pathway [GO:0017015]; is a type of positive regulation of transmembrane receptor protein serine/threonine kinase signaling pathway [GO:0090100]; is a type of positive regulation of cellular response to transforming growth factor beta stimulus [GO:1903846]; positively regulates transforming growth factor beta receptor signaling pathway [GO:0007179] Also known as: positive regulation of TGF-beta receptor signaling pathway, positive regulation of TGFbeta receptor signaling pathway, positive regulation of transforming growth factor beta receptor signalling pathway, up regulation of transforming growth factor beta receptor signaling pathway, up-regulation of transforming growth factor beta receptor signaling pathway, upregulation of transforming growth factor beta receptor signaling pathway, activation of transforming growth factor beta receptor signaling pathway, stimulation of transforming growth factor beta receptor signaling pathway